{
  "gene": "UniProtKB:Q6JHZ5",
  "gene_symbol": "Q6JHZ5",
  "term_id": "UNKNOWN:0002",
  "term_label": "Unknown biological process",
  "gene_name": "NS5ATP13TP1"
}